{
  "gene_name": "Polymerase delta-interacting protein 3",
  "gene_symbol": "POLDIP3",
  "term_id": "GO:0005634",
  "term_label": "nucleus",
  "gene": "UniProtKB:Q9BY77"
}